chromosome organization involved in meiotic cell cycle [GO:0070192] (biological process) Relationships: is a type of chromosome organization [GO:0051276]; is_a GO:1903046 Subtypes: homologous chromosome pairing at meiosis [GO:0007129], synaptonemal complex assembly [GO:0007130], GO:0010032, meiotic telomere clustering [GO:0045141], meiotic sister chromatid segregation [GO:0045144], karyosome formation [GO:0061988], linear element maturation [GO:0062121], GO:0106212, kinetochore disassembly involved in meiotic chromosome organization [GO:0106213], meiotic telomere maintenance via semi-conservative replication [GO:1902989], meiotic centromere clustering [GO:1990571] Also known as: chromosome organisation involved in meiosis, meiotic chromosome organization Definition: A process of chromosome organization that is involved in a meiotic cell cycle. Sources: GOC:mah